negative regulation of cuticle pigmentation [GO:0048080] (biological process) Definition: Any process that stops, prevents, or reduces the frequency, rate or extent of establishment of a pattern of pigment in the cuticle of an organism. Subtypes: GO:0048083 Also known as: down regulation of cuticle pigmentation, down-regulation of cuticle pigmentation, downregulation of cuticle pigmentation, inhibition of cuticle pigmentation Sources: GOC:jid Relationships: is a type of GO:0048079; is a type of GO:0048086; is a type of negative regulation of developmental process [GO:0051093]; is a type of negative regulation of multicellular organismal process [GO:0051241]; negatively regulates GO:0048067